{
  "term_label": "negative regulation of B cell proliferation",
  "gene": "UniProtKB:O43914",
  "term_id": "GO:0030889",
  "gene_name": "TYRO protein tyrosine kinase-binding protein",
  "gene_symbol": "TYROBP"
}